{
  "gene": "UniProtKB:O95436",
  "term_label": "vesicle",
  "gene_name": "Sodium-dependent phosphate transport protein 2B",
  "term_id": "GO:0031982",
  "gene_symbol": "SLC34A2"
}